spindle assembly involved in male meiosis II [GO:0007055] (biological process) Definition: The formation of the spindle during meiosis II of a meiotic cell cycle in males. An example of this is found in Drosophila melanogaster. Sources: GOC:mah Also known as: male meiosis II spindle assembly Relationships: is a type of spindle assembly involved in male meiosis [GO:0007053]; BFO_0000050 male meiosis II [GO:0007142]